{
  "gene_symbol": "HOXA13",
  "gene_name": "Homeobox protein Hox-A13",
  "term_id": "UNKNOWN:0003",
  "gene": "UniProtKB:P31271",
  "term_label": "Unknown cellular component"
}